{
  "gene_name": "Poly(A) polymerase beta",
  "gene": "UniProtKB:Q9NRJ5",
  "term_label": "nucleus",
  "term_id": "GO:0005634",
  "gene_symbol": "PAPOLB"
}